{
  "term_id": "GO:0032418",
  "term_label": "lysosome localization",
  "gene": "UniProtKB:Q9BQD3",
  "gene_name": "KxDL motif-containing protein 1",
  "gene_symbol": "KXD1"
}